{
  "term_id": "GO:1990138",
  "gene": "UniProtKB:Q496H8",
  "gene_name": "Neuritin-like protein",
  "term_label": "neuron projection extension",
  "gene_symbol": "NRN1L"
}